{
  "gene_name": "Pre-mRNA-splicing factor CWC25 homolog",
  "term_label": "U2-type spliceosomal complex",
  "gene": "UniProtKB:Q9NXE8",
  "gene_symbol": "CWC25",
  "term_id": "GO:0005684"
}